regulation of pH [GO:0006885] (biological process) Also known as: hydrogen ion homeostasis Sources: GOC:dph, GOC:go_curators, GOC:tb Relationships: is a type of monoatomic cation homeostasis [GO:0055080]; is a type of biological regulation [GO:0065007] Subtypes: GO:0030641, pH reduction [GO:0045851], pH elevation [GO:0045852] Definition: Any process involved in the maintenance of an internal equilibrium of hydrogen ions, thereby modulating the internal pH, within an organism or cell.